{
  "gene": "UniProtKB:Q8N4T4",
  "gene_symbol": "ARHGEF39",
  "term_id": "GO:0030335",
  "term_label": "positive regulation of cell migration",
  "gene_name": "Rho guanine nucleotide exchange factor 39"
}